{
  "term_label": "regulation of mitotic nuclear division",
  "gene": "UniProtKB:Q4G163",
  "term_id": "GO:0007088",
  "gene_name": "F-box only protein 43",
  "gene_symbol": "FBXO43"
}